{
  "term_label": "nucleotide-excision repair",
  "gene": "UniProtKB:Q13888",
  "term_id": "GO:0006289",
  "gene_name": "General transcription factor IIH subunit 2",
  "gene_symbol": "GTF2H2"
}